{
  "gene_symbol": "LSM4",
  "gene_name": "U6 snRNA-associated Sm-like protein LSm4",
  "gene": "UniProtKB:Q9Y4Z0",
  "term_label": "spliceosomal snRNP assembly",
  "term_id": "GO:0000387"
}